{
  "gene_symbol": "PLSCR3",
  "gene_name": "Phospholipid scramblase 3",
  "term_label": "plasma membrane",
  "term_id": "GO:0005886",
  "gene": "UniProtKB:Q9NRY6"
}